{
  "gene_symbol": "SPATA16",
  "term_id": "GO:0007283",
  "gene_name": "Spermatogenesis-associated protein 16",
  "gene": "UniProtKB:Q9BXB7",
  "term_label": "spermatogenesis"
}